{
  "gene": "UniProtKB:Q01064",
  "term_id": "GO:0048101",
  "gene_symbol": "PDE1B",
  "gene_name": "Dual specificity calcium_calmodulin-dependent 3',5'-cyclic nucleotide phosphodiesterase 1B",
  "term_label": "calmodulin-activated 3',5'-cyclic-GMP phosphodiesterase activity"
}